negative regulation of nephron tubule epithelial cell differentiation [GO:0072183] (biological process) Sources: GOC:mtg_kidney_jan10 Definition: Any process that decreases the frequency, rate or extent of nephron tubule epithelial cell differentiation. Subtypes: negative regulation of metanephric nephron tubule epithelial cell differentiation [GO:0072308], GO:2000094 Relationships: is a type of regulation of nephron tubule epithelial cell differentiation [GO:0072182]; is a type of negative regulation of kidney development [GO:0090185]; is a type of negative regulation of epithelial cell differentiation involved in kidney development [GO:2000697]; negatively regulates nephron tubule epithelial cell differentiation [GO:0072160]